{
  "term_label": "Unknown molecular function",
  "gene_name": "Membrane-spanning 4-domains subfamily A member 12",
  "term_id": "UNKNOWN:0001",
  "gene": "UniProtKB:Q9NXJ0",
  "gene_symbol": "MS4A12"
}